{
  "gene": "UniProtKB:Q9UGP4",
  "term_label": "P-body",
  "gene_symbol": "LIMD1",
  "gene_name": "LIM domain-containing protein 1",
  "term_id": "GO:0000932"
}